{
  "gene_symbol": "LXN",
  "gene": "UniProtKB:Q9BS40",
  "term_id": "UNKNOWN:0002",
  "term_label": "Unknown biological process",
  "gene_name": "Latexin"
}